dosage compensation by hyperactivation of X chromosome [GO:0009047] (biological process) Definition: Compensating for the two-fold variation in X-chromosome:autosome ratios between sexes by a global hyperactivation of all, or most of, the genes on the X-chromosome in the heterogametic sex, leading to a two-fold increase in gene expression from this chromosome. An example of this is found in Drosophila melanogaster. Relationships: is a type of sex-chromosome dosage compensation [GO:0007549] References: PMID:11498577, PMID:1568251 Sources: GOC:jl, GOC:mr